{
  "term_id": "GO:0016559",
  "gene": "UniProtKB:O00429",
  "term_label": "peroxisome fission",
  "gene_name": "Dynamin-1-like protein",
  "gene_symbol": "DNM1L"
}